2-methylbut-2-enoyl-CoA(4-) metabolic process [GO:1902192] (biological process) Subtypes: 2-methylbut-2-enoyl-CoA(4-) catabolic process [GO:1902193], 2-methylbut-2-enoyl-CoA(4-) biosynthetic process [GO:1902194] Definition: The chemical reactions and pathways involving 2-methylbut-2-enoyl-CoA(4-). Relationships: is a type of fatty-acyl-CoA metabolic process [GO:0035337] References: PMID:15574432 Sources: GOC:TermGenie Also known as: 2-methylbut-2-enoyl-CoA(4-) metabolism